{
  "term_id": "GO:0006805",
  "gene_symbol": "GSTA4",
  "gene_name": "Glutathione S-transferase A4",
  "gene": "UniProtKB:O15217",
  "term_label": "xenobiotic metabolic process"
}